{
  "gene_name": "Endoplasmic reticulum resident protein 29",
  "gene": "UniProtKB:P30040",
  "term_label": "Unknown biological process",
  "gene_symbol": "ERP29",
  "term_id": "UNKNOWN:0002"
}